{
  "gene_symbol": "TRAF7",
  "gene_name": "E3 ubiquitin-protein ligase TRAF7",
  "term_label": "positive regulation of MAPK cascade",
  "gene": "UniProtKB:Q6Q0C0",
  "term_id": "GO:0043410"
}